{
  "term_label": "regulation of membrane potential",
  "gene": "UniProtKB:Q9HBV1",
  "gene_name": "Popeye domain-containing protein 3",
  "term_id": "GO:0042391",
  "gene_symbol": "POPDC3"
}